{
  "gene_symbol": "IL1RAPL2",
  "term_label": "cell surface",
  "gene_name": "X-linked interleukin-1 receptor accessory protein-like 2",
  "term_id": "GO:0009986",
  "gene": "UniProtKB:Q9NP60"
}